{
  "gene_symbol": "TEX50",
  "term_id": "UNKNOWN:0001",
  "gene": "UniProtKB:A0A1B0GTY4",
  "term_label": "Unknown molecular function",
  "gene_name": "Testis-expressed protein 50"
}